XTP binding [GO:1901640] (molecular function) Definition: Binding to XTP. Relationships: is a type of purine ribonucleotide binding [GO:0032555]; is a type of purine ribonucleoside triphosphate binding [GO:0035639] Sources: GOC:TermGenie